positive regulation of maltohexaose transport [GO:1900314] (biological process) Definition: Any process that activates or increases the frequency, rate or extent of maltohexaose transport. Also known as: up regulation of maltohexaose transport, up-regulation of maltohexaose transport, upregulation of maltohexaose transport, activation of maltohexaose transport Sources: GOC:TermGenie, GOC:mengo_curators Relationships: is a type of positive regulation of hexasaccharide transport [GO:1900299]; is_a GO:1900312; positively regulates maltohexaose transport [GO:2001103]